{
  "term_id": "GO:0005886",
  "gene": "UniProtKB:Q9Y5X5",
  "gene_name": "Neuropeptide FF receptor 2",
  "gene_symbol": "NPFFR2",
  "term_label": "plasma membrane"
}